{
  "term_id": "UNKNOWN:0002",
  "gene_symbol": "A0A6Q8PGZ7",
  "gene_name": "Uncharacterized protein",
  "term_label": "Unknown biological process",
  "gene": "UniProtKB:A0A6Q8PGZ7"
}